icosanoid secretion [GO:0032309] (biological process) Subtypes: prostaglandin secretion [GO:0032310], GO:0050482 Also known as: eicosanoid secretion Sources: GOC:mah Relationships: is a type of secretion [GO:0046903]; is a type of icosanoid transport [GO:0071715] Regulation: regulated by regulation of icosanoid secretion [GO:0032303]; negatively regulated by GO:0032304; positively regulated by positive regulation of icosanoid secretion [GO:0032305] Definition: The controlled release of icosanoids, any of a group of C20 polyunsaturated fatty acids from a cell or a tissue.